{
  "gene_name": "Transcription factor GATA-4",
  "gene": "UniProtKB:P43694",
  "term_label": "DNA-binding transcription factor activity, RNA polymerase II-specific",
  "gene_symbol": "GATA4",
  "term_id": "GO:0000981"
}